{
  "term_id": "GO:0005737",
  "term_label": "cytoplasm",
  "gene_name": "Glutathione S-transferase theta-1",
  "gene_symbol": "GSTT1",
  "gene": "UniProtKB:P30711"
}